regulation of hippo signaling [GO:0035330] (biological process) Subtypes: negative regulation of hippo signaling [GO:0035331], positive regulation of hippo signaling [GO:0035332] Sources: GOC:bf Relationships: is a type of regulation of intracellular signal transduction [GO:1902531]; regulates GO:0035329 Definition: Any process that modulates the frequency, rate or extent of hippo signaling. Also known as: regulation of hippo signaling pathway, regulation of hippo signaling cascade, regulation of hippo signalling cascade